{
  "gene_name": "mRNA decay activator protein ZFP36L1",
  "term_label": "protein-RNA sequence-specific adaptor activity",
  "gene": "UniProtKB:Q07352",
  "term_id": "GO:0160134",
  "gene_symbol": "ZFP36L1"
}